{
  "term_label": "Unknown molecular function",
  "term_id": "UNKNOWN:0001",
  "gene_symbol": "GLIPR1L2",
  "gene": "UniProtKB:Q4G1C9",
  "gene_name": "GLIPR1-like protein 2"
}